{
  "gene_symbol": "JMJD1C",
  "gene": "UniProtKB:Q15652",
  "gene_name": "Probable JmjC domain-containing histone demethylation protein 2C",
  "term_label": "chromatin DNA binding",
  "term_id": "GO:0031490"
}